{
  "gene": "UniProtKB:O60522",
  "gene_symbol": "TDRD6",
  "gene_name": "Tudor domain-containing protein 6",
  "term_label": "Unknown molecular function",
  "term_id": "UNKNOWN:0001"
}